lumenal side of endosome membrane [GO:0098565] (cellular component) Also known as: internal leaflet of endosome membrane, internal side of endosome membrane Subtypes: lumenal side of early endosome membrane [GO:0098550], GO:0098551 Sources: GOC:dos Relationships: is a type of lumenal side of membrane [GO:0098576]; is part of endosome membrane [GO:0010008] Definition: The side (leaflet) of the endosome membrane that faces the lumen.